{
  "term_label": "nucleus",
  "term_id": "GO:0005634",
  "gene": "UniProtKB:Q9BWX1",
  "gene_symbol": "PHF7",
  "gene_name": "PHD finger protein 7"
}